{
  "gene_name": "Olfactory receptor 2T11",
  "gene": "UniProtKB:Q8NH01",
  "gene_symbol": "OR2T11",
  "term_id": "GO:0050911",
  "term_label": "detection of chemical stimulus involved in sensory perception of smell"
}